inhibition of epinephrine uptake [GO:0051629] (biological process) Also known as: inhibition of adrenaline uptake, inhibition of epinephrine import Relationships: is a type of inhibition of neurotransmitter uptake [GO:0051609]; is a type of negative regulation of epinephrine uptake [GO:0051627] Definition: Any process that prevents the activation of the directed movement of epinephrine into a cell. Sources: GOC:ai